receptor complex [GO:0043235] (cellular component) Subtypes: GO:0002116, tumor necrosis factor receptor superfamily complex [GO:0002947], aryl hydrocarbon receptor complex [GO:0034751], GO:0035692, GO:0038104, GO:0046696, growth hormone receptor complex [GO:0070195], serotonin receptor complex [GO:0098665], G protein-coupled serotonin receptor complex [GO:0098666], plasma membrane signaling receptor complex [GO:0098802], decoy receptor complex [GO:0140368], GABA receptor complex [GO:1902710], taste receptor complex [GO:1903768], interleukin-7 receptor complex [GO:1905540], interleukin-15 receptor complex [GO:1905543], interleukin-10 receptor complex [GO:1905571], GO:1990620 Definition: Any protein complex that undergoes combination with a hormone, neurotransmitter, drug or intracellular messenger to initiate a change in cell function. Sources: GOC:go_curators Relationships: is a type of protein-containing complex [GO:0032991]